{
  "term_label": "ubiquitin ligase complex",
  "term_id": "GO:0000151",
  "gene_symbol": "DCUN1D5",
  "gene_name": "DCN1-like protein 5",
  "gene": "UniProtKB:Q9BTE7"
}